{
  "term_label": "DNA-binding transcription factor activity, RNA polymerase II-specific",
  "term_id": "GO:0000981",
  "gene_symbol": "ZNF253",
  "gene": "UniProtKB:O75346",
  "gene_name": "Zinc finger protein 253"
}